{
  "gene": "UniProtKB:A6NGC4",
  "term_label": "membrane assembly",
  "gene_name": "TLC domain-containing protein 2",
  "term_id": "GO:0071709",
  "gene_symbol": "TLCD2"
}